{
  "term_label": "Unknown biological process",
  "gene_symbol": "OR11H4",
  "gene_name": "Olfactory receptor 11H4",
  "gene": "UniProtKB:Q8NGC9",
  "term_id": "UNKNOWN:0002"
}